{
  "gene_symbol": "UTF1",
  "gene": "UniProtKB:Q5T230",
  "term_label": "transcription coactivator activity",
  "gene_name": "Undifferentiated embryonic cell transcription factor 1",
  "term_id": "GO:0003713"
}